negative regulation of ethylene-activated signaling pathway [GO:0010105] (biological process) Definition: Any process that stops or prevents ethylene (ethene) signal transduction. Sources: GOC:tb Also known as: down regulation of ethylene mediated signaling pathway, down-regulation of ethylene mediated signaling pathway, downregulation of ethylene mediated signaling pathway, negative regulation of ethene mediated signaling pathway, negative regulation of ethene mediated signalling pathway, negative regulation of ethylene mediated signalling pathway, inhibition of ethylene mediated signaling pathway, negative regulation of ethylene mediated signaling pathway Relationships: is a type of regulation of ethylene-activated signaling pathway [GO:0010104]; is a type of negative regulation of phosphorelay signal transduction system [GO:0070298]; negatively regulates ethylene-activated signaling pathway [GO:0009873]